cardiac endothelial cell differentiation [GO:0003348] (biological process) Definition: The process in which a relatively unspecialized cell acquires the specialized structural and/or functional features of a cardiac endothelial cell. Relationships: is_a cardiocyte differentiation [GO:0035051]; is a type of GO:0045446 Subtypes: epicardium-derived cardiac endothelial cell differentiation [GO:0003349], cardiac blood vessel endothelial cell differentiation [GO:0060946], GO:0060956 References: PMID:18722343 Sources: GOC:dph